{
  "term_label": "microtubule binding",
  "gene": "UniProtKB:O15182",
  "term_id": "GO:0008017",
  "gene_symbol": "CETN3",
  "gene_name": "Centrin-3"
}